{
  "gene_name": "Thyroglobulin",
  "term_id": "GO:0006590",
  "gene": "UniProtKB:P01266",
  "term_label": "thyroid hormone generation",
  "gene_symbol": "TG"
}